linolenate 9R-lipoxygenase activity [GO:0102299] (molecular function) Definition: Catalysis of the reaction: (9Z,12Z,15Z)-octadecatrienoate + O2 = (9R,10E,12Z,15Z)-9-hydroperoxyoctadeca-10,12,15-trienoate. Also converts linoleate to (9R,10E,12Z)-9- hydroperoxyoctadeca-10,12-dienoate. Sources: EC:1.13.11.61 Relationships: is a type of oxidoreductase activity, acting on single donors with incorporation of molecular oxygen, incorporation of two atoms of oxygen [GO:0016702]